1-alkyl-2-acetylglycerophosphocholine esterase complex [GO:0008247] (cellular component) References: PMID:10542206 Sources: GOC:jl Also known as: 2-acetyl-1-alkylglycerophosphocholine esterase complex, platelet-activating factor acetylhydrolase complex Definition: An enzyme complex composed of two catalytic alpha subunits, which form a catalytic dimer, and a non-catalytic, regulatory beta subunit; the catalytic dimer may be an alpha1/alpha1 or alpha2/alpha2 homodimer, or an alpha1/alpha2 heterodimer. Modulates the action of platelet-activating factor (PAF). Relationships: is a type of catalytic complex [GO:1902494] Note: See also the molecular function term '1-alkyl-2-acetylglycerophosphocholine esterase activity ; GO:0003847'.